{
  "gene_symbol": "AKAP9",
  "gene_name": "A-kinase anchor protein 9",
  "gene": "UniProtKB:Q99996",
  "term_label": "Golgi stack",
  "term_id": "GO:0005795"
}